{
  "term_id": "GO:0030246",
  "gene": "UniProtKB:P56470",
  "gene_symbol": "LGALS4",
  "gene_name": "Galectin-4",
  "term_label": "carbohydrate binding"
}